glyceraldehyde dehydrogenase (NADP+) activity [GO:0043796] (molecular function) Relationships: is a type of GO:0033721 Sources: RHEA:40163 Definition: Catalysis of the reaction: D-glyceraldehyde + H2O + NADP+ = D-glycerate + NADPH + H+. Also known as: glyceraldehyde dehydrogenase (NADP) activity